{
  "gene_name": "Lysosomal-associated transmembrane protein 5",
  "term_label": "protein sequestering activity",
  "gene_symbol": "LAPTM5",
  "term_id": "GO:0140311",
  "gene": "UniProtKB:Q13571"
}